{
  "gene": "UniProtKB:P00568",
  "term_id": "GO:0005737",
  "gene_symbol": "AK1",
  "gene_name": "Adenylate kinase isoenzyme 1",
  "term_label": "cytoplasm"
}